copper ion transmembrane transporter activity [GO:0005375] (molecular function) Relationships: is_a transition metal ion transmembrane transporter activity [GO:0046915]; is part of copper ion transmembrane transport [GO:0035434] Definition: Enables the transfer of copper (Cu) ions from one side of a membrane to the other. Subtypes: high-affinity copper ion transmembrane transporter activity [GO:0015089], P-type divalent copper transporter activity [GO:0043682], copper chelate transmembrane transporter activity [GO:0051981], GO:0140581 Also known as: intracellular copper ion transporter, plasma membrane copper transporter, copper uptake transmembrane transporter activity Sources: GOC:ai